integrin alphav-beta1 complex [GO:0034682] (cellular component) Relationships: is a type of integrin complex [GO:0008305] Definition: An integrin complex that comprises one alphav subunit and one beta1 subunit. Also known as: alphav-beta1 integrin complex, ITGAV-ITGB1 complex References: PMID:12297042